glycerol-3-phosphate cytidylyltransferase activity [GO:0047348] (molecular function) Definition: Catalysis of the reaction: sn-glycerol 3-phosphate + CTP = CDP-glycerol + diphosphate. Relationships: is a type of cytidylyltransferase activity [GO:0070567] Sources: RHEA:13361 Also known as: CTP:glycerol-3-phosphate cytidylyltransferase activity, CDP-glycerol diphosphorylase activity, CDP-glycerol pyrophosphorylase activity, CTP:glycerol 3-phosphate cytidylyltransferase activity, CTP:sn-glycerol-3-phosphate cytidylyltransferase activity, Gro-PCT, cytidine diphosphate glycerol pyrophosphorylase activity, cytidine diphosphoglycerol pyrophosphorylase activity